{
  "gene": "UniProtKB:Q6UXT9",
  "term_label": "lipid metabolic process",
  "gene_symbol": "ABHD15",
  "term_id": "GO:0006629",
  "gene_name": "Protein ABHD15"
}